{
  "term_label": "multivesicular body",
  "gene_symbol": "CHMP7",
  "gene_name": "Charged multivesicular body protein 7",
  "gene": "UniProtKB:Q8WUX9",
  "term_id": "GO:0005771"
}